phospholipase C-activating endothelin receptor signaling pathway [GO:0160135] (biological process) Relationships: is a type of phospholipase C-activating G protein-coupled receptor signaling pathway [GO:0007200]; is a type of endothelin receptor signaling pathway [GO:0086100] References: PMID:35284927 Definition: A phospholipase C-activating receptor G protein-coupled receptor signaling pathway initiated by endothelin binding to its receptor on the surface of a target cell, and ending with the regulation of a downstream cellular process, e.g. transcription.